{
  "gene_symbol": "NOS3",
  "term_id": "GO:0005886",
  "gene": "UniProtKB:P29474",
  "gene_name": "Nitric oxide synthase 3",
  "term_label": "plasma membrane"
}